detection of mechanical stimulus involved in magnetoreception [GO:0050971] (biological process) Relationships: is a type of detection of mechanical stimulus involved in sensory perception [GO:0050974]; is part of GO:0050979 Sources: GOC:ai, GOC:dos Definition: The series of events involved in magnetoception in which a mechanical stimulus is received and converted into a molecular signal. The stimulus is in the form of torque on particles such as magnetite which respond to a magnetic field. Also known as: magnetoception, sensory transduction of mechanical stimulus, magnetoreception, detection of mechanical stimulus, magnetoreception, sensory detection of mechanical stimulus, magnetoreception, sensory transduction of mechanical stimulus, sensory detection of mechanical stimulus during magnetoreception, sensory transduction of mechanical stimulus during magnetoreception